{
  "term_id": "UNKNOWN:0002",
  "gene_name": "Trans-3-hydroxy-L-proline dehydratase",
  "gene": "UniProtKB:Q96EM0",
  "gene_symbol": "L3HYPDH",
  "term_label": "Unknown biological process"
}